prostaglandin F receptor activity [GO:0004958] (molecular function) Also known as: PGF(2-alpha) receptor activity, PGF receptor activity Sources: ISBN:0198506732 Definition: Combining with prostaglandin F (PGF (2-alpha)) to initiate a change in cell activity. Relationships: is a type of prostaglandin receptor activity [GO:0004955]